{
  "term_label": "extracellular space",
  "gene": "UniProtKB:P22301",
  "term_id": "GO:0005615",
  "gene_name": "Interleukin-10",
  "gene_symbol": "IL10"
}